{
  "term_id": "GO:0061844",
  "gene": "UniProtKB:P47992",
  "gene_name": "Lymphotactin",
  "term_label": "antimicrobial humoral immune response mediated by antimicrobial peptide",
  "gene_symbol": "XCL1"
}